{
  "gene_symbol": "DHRS4L1",
  "gene": "UniProtKB:P0CG22",
  "term_id": "GO:0004090",
  "gene_name": "Putative dehydrogenase_reductase SDR family member 4-like 1",
  "term_label": "carbonyl reductase (NADPH) activity"
}